{
  "term_id": "GO:0048858",
  "gene_name": "Ras-associated and pleckstrin homology domains-containing protein 1",
  "gene_symbol": "RAPH1",
  "gene": "UniProtKB:Q70E73",
  "term_label": "cell projection morphogenesis"
}